lactose:proton symporter activity [GO:0015528] (molecular function) Sources: TC:2.A.1.1.9, TC:2.A.1.5.1 Definition: Enables the transfer of a solute or solutes from one side of a membrane to the other according to the reaction: lactose(out) + H+(out) = lactose(in) + H+(in). Relationships: is a type of GO:0005351; is a type of lactose transmembrane transporter activity [GO:0015155] Also known as: lactose, galactose:hydrogen symporter activity, lactose:hydrogen symporter activity